{
  "term_id": "UNKNOWN:0001",
  "term_label": "Unknown molecular function",
  "gene": "UniProtKB:Q9H9Y6",
  "gene_name": "DNA-directed RNA polymerase I subunit RPA2",
  "gene_symbol": "POLR1B"
}